{
  "gene_name": "Immunoglobulin heavy variable 4-34",
  "gene": "UniProtKB:P06331",
  "term_label": "immunoglobulin mediated immune response",
  "gene_symbol": "IGHV4-34",
  "term_id": "GO:0016064"
}